phosphoenolpyruvate transmembrane transporter activity [GO:0089721] (molecular function) Subtypes: GO:0015121 Relationships: is a type of monocarboxylic acid transmembrane transporter activity [GO:0008028]; is_a organophosphate ester transmembrane transporter activity [GO:0015605]; BFO_0000050 phosphoenolpyruvate transmembrane transport [GO:0089722] Sources: GOC:dos Definition: Enables the transfer of a phosphoenolpyruvate from one side of a membrane to the other.